{
  "gene": "UniProtKB:Q8N3X6",
  "term_label": "nucleus",
  "gene_symbol": "LCORL",
  "term_id": "GO:0005634",
  "gene_name": "Ligand-dependent nuclear receptor corepressor-like protein"
}